{
  "gene_name": "BH3-like motif-containing cell death inducer",
  "term_id": "UNKNOWN:0003",
  "term_label": "Unknown cellular component",
  "gene": "UniProtKB:Q8IZY5",
  "gene_symbol": "BLID"
}